positive regulation of RNA metabolic process [GO:0051254] (biological process) Subtypes: positive regulation of mitochondrial RNA catabolic process [GO:0000962], GO:0050779, positive regulation of RNA biosynthetic process [GO:1902680], positive regulation of mRNA metabolic process [GO:1903313], positive regulation of snoRNA metabolic process [GO:1903325], positive regulation of tRNA metabolic process [GO:1903328], positive regulation of snRNA pseudouridine synthesis [GO:1905358], positive regulation of rRNA processing [GO:2000234], positive regulation of miRNA metabolic process [GO:2000630] Definition: Any process that activates or increases the frequency, rate or extent of the chemical reactions and pathways involving RNA. Sources: GOC:ai Relationships: is a type of positive regulation of macromolecule metabolic process [GO:0010604]; is a type of GO:0051252; positively regulates RNA metabolic process [GO:0016070] Also known as: positive regulation of RNA metabolism, up regulation of RNA metabolic process, up-regulation of RNA metabolic process, upregulation of RNA metabolic process, activation of RNA metabolic process, stimulation of RNA metabolic process